{
  "term_id": "GO:0030175",
  "gene_symbol": "PALM",
  "gene": "UniProtKB:O75781",
  "term_label": "filopodium",
  "gene_name": "Paralemmin-1"
}